{
  "gene_name": "Beta-soluble NSF attachment protein",
  "term_id": "GO:0005483",
  "gene": "UniProtKB:Q9H115",
  "term_label": "soluble NSF attachment protein activity",
  "gene_symbol": "NAPB"
}